type III polyketide synthase complex [GO:0034083] (cellular component) Also known as: type III PKS, type III PKS complex, type III polyketide synthase Relationships: is a type of polyketide synthase complex [GO:0034081] References: PMID:12636085 Sources: GOC:cb Definition: A polyketide synthase complex that consists of two identical ketosynthase polypeptides.